negative regulation of glial cell differentiation [GO:0045686] (biological process) Relationships: is a type of negative regulation of gliogenesis [GO:0014014]; is_a regulation of glial cell differentiation [GO:0045685]; negatively regulates glial cell differentiation [GO:0010001] Subtypes: negative regulation of microglia differentiation [GO:0014007], negative regulation of Schwann cell differentiation [GO:0014039], negative regulation of astrocyte differentiation [GO:0048712], negative regulation of oligodendrocyte differentiation [GO:0048715] Also known as: down regulation of glial cell differentiation, down-regulation of glial cell differentiation, downregulation of glial cell differentiation, negative regulation of glia cell differentiation, negative regulation of neuroglia differentiation, inhibition of glial cell differentiation Sources: GOC:go_curators Definition: Any process that stops, prevents, or reduces the frequency, rate or extent of glia cell differentiation.